{
  "gene_name": "Proto-oncogene vav",
  "term_label": "positive regulation of phosphatidylinositol 3-kinase/protein kinase B signal transduction",
  "term_id": "GO:0051897",
  "gene_symbol": "VAV1",
  "gene": "UniProtKB:P15498"
}